{
  "gene_symbol": "KRTAP7-1",
  "gene": "UniProtKB:Q8IUC3",
  "term_id": "UNKNOWN:0002",
  "gene_name": "Keratin-associated protein 7-1",
  "term_label": "Unknown biological process"
}